alkanesulfonate monooxygenase activity [GO:0008726] (molecular function) Also known as: FMNH(2)-dependent alkanesulfonate monooxygenase activity, alkanesulphonate monooxygenase activity, FMNH(2)-dependent aliphatic sulfonate monooxygenase activity, FMNH2-dependent aliphatic sulfonate monooxygenase activity, SsuD, alkanesulfonate, reduced-FMN:oxygen oxidoreductase activity, sulfate starvation-induced protein 6 activity Sources: MetaCyc:RXN0-280 Definition: Catalysis of the reaction: an alkanesulfonate + O2 + FMNH2 = an aldehyde + sulfite + H2O + FMN. Relationships: is a type of oxidoreductase activity, acting on paired donors, with incorporation or reduction of molecular oxygen, reduced flavin or flavoprotein as one donor, and incorporation of one atom of oxygen [GO:0016712]